cell wall macromolecule catabolic process [GO:0016998] (biological process) Definition: The chemical reactions and pathways resulting in the breakdown of macromolecules that form part of a cell wall. Sources: GOC:go_curators Also known as: cellular cell wall macromolecule breakdown, cellular cell wall macromolecule catabolic process, cellular cell wall macromolecule catabolism, cellular cell wall macromolecule degradation, cell wall breakdown, cell wall catabolism, cell wall degradation Relationships: is a type of macromolecule catabolic process [GO:0009057]; is a type of cell wall macromolecule metabolic process [GO:0044036] Subtypes: cell wall macromolecule catabolic process involved in cytogamy [GO:0032219], cell wall polysaccharide catabolic process [GO:0044347], wall teichoic acid catabolic process [GO:0070399], cell wall macromolecule catabolic process involved in cell wall disassembly [GO:0070910]